{
  "term_id": "GO:0043171",
  "gene": "UniProtKB:P09960",
  "term_label": "peptide catabolic process",
  "gene_symbol": "LTA4H",
  "gene_name": "Leukotriene A-4 hydrolase"
}